{
  "gene_name": "Platelet-derived growth factor D",
  "term_label": "extracellular space",
  "term_id": "GO:0005615",
  "gene_symbol": "PDGFD",
  "gene": "UniProtKB:Q9GZP0"
}